positive regulation of triglyceride storage [GO:0010890] (biological process) Also known as: positive regulation of sequestering of triacylglycerol, positive regulation of sequestering of triglyceride, positive regulation of triglyceride sequestration Relationships: is a type of positive regulation of lipid storage [GO:0010884]; is a type of regulation of triglyceride storage [GO:0010889]; positively regulates GO:0030730 Sources: GOC:BHF, GOC:dph, GOC:tb Definition: Any process that increases the rate, frequency or extent of sequestering of triglyceride. Triglyceride sequestration is the process of binding or confining any triester of glycerol such that it is separated from other components of a biological system.